{
  "gene": "UniProtKB:O43915",
  "term_id": "GO:0038084",
  "term_label": "vascular endothelial growth factor signaling pathway",
  "gene_symbol": "VEGFD",
  "gene_name": "Vascular endothelial growth factor D"
}